{
  "gene_name": "Melanoma-associated antigen B6",
  "term_id": "GO:0005634",
  "gene_symbol": "MAGEB6",
  "gene": "UniProtKB:Q8N7X4",
  "term_label": "nucleus"
}